{
  "gene": "UniProtKB:Q5VSL9",
  "gene_symbol": "STRIP1",
  "term_label": "FAR/SIN/STRIPAK complex",
  "term_id": "GO:0090443",
  "gene_name": "Striatin-interacting protein 1"
}